{
  "term_label": "RNA polymerase II cis-regulatory region sequence-specific DNA binding",
  "gene": "UniProtKB:Q9NP71",
  "term_id": "GO:0000978",
  "gene_name": "Carbohydrate-responsive element-binding protein",
  "gene_symbol": "MLXIPL"
}